{
  "term_id": "GO:0061656",
  "gene": "UniProtKB:P63279",
  "gene_name": "SUMO-conjugating enzyme UBC9",
  "gene_symbol": "UBE2I",
  "term_label": "SUMO conjugating enzyme activity"
}